phenylacetaldehyde dehydrogenase (NAD+) activity [GO:0008957] (molecular function) Relationships: is_a GO:0004029 Also known as: phenylacetaldehyde:NAD+ oxidoreductase activity Sources: RHEA:21392 Definition: Catalysis of the reaction: 2-phenylacetaldehyde + H2O + NAD+ = 2-phenylacetate + 2 H+ + NADH.